{
  "gene_symbol": "GSR",
  "term_id": "GO:0005739",
  "gene_name": "Glutathione reductase, mitochondrial",
  "gene": "UniProtKB:P00390",
  "term_label": "mitochondrion"
}